regulation of neuronal signal transduction [GO:1902847] (biological process) Subtypes: GO:1902848, GO:1902849 Sources: GOC:TermGenie, GOC:sjp, GO_REF:0000058 Definition: Any process that modulates the frequency, rate or extent of neuronal signal transduction. Relationships: is a type of regulation of signal transduction [GO:0009966]; regulates neuronal signal transduction [GO:0023041]